regulation of emodin biosynthetic process [GO:1900664] (biological process) Definition: Any process that modulates the frequency, rate or extent of emodin biosynthetic process. Relationships: is a type of regulation of ketone biosynthetic process [GO:0010566]; is a type of regulation of secondary metabolite biosynthetic process [GO:1900376]; RO_0002211 emodin biosynthetic process [GO:1900575] Sources: GOC:TermGenie, GOC:di Also known as: regulation of emodin anabolism, regulation of emodin biosynthesis, regulation of emodin formation, regulation of emodin synthesis Subtypes: negative regulation of emodin biosynthetic process [GO:1900665], positive regulation of emodin biosynthetic process [GO:1900666]